{
  "term_label": "mitochondrion",
  "gene_symbol": "DNLZ",
  "gene": "UniProtKB:Q5SXM8",
  "gene_name": "DNL-type zinc finger protein",
  "term_id": "GO:0005739"
}